{
  "gene_name": "rRNA-processing protein UTP23 homolog",
  "gene_symbol": "UTP23",
  "term_label": "Unknown biological process",
  "term_id": "UNKNOWN:0002",
  "gene": "UniProtKB:Q9BRU9"
}